1,2-dehydroreticulinium reductase (NADPH) activity [GO:0047128] (molecular function) Sources: EC:1.5.1.27, RHEA:17569 Also known as: (R)-reticuline:NADP+ oxidoreductase activity, 1,2-dehydroreticulinium ion reductase activity Relationships: is a type of oxidoreductase activity, acting on the CH-NH group of donors, NAD or NADP as acceptor [GO:0016646] Definition: Catalysis of the reaction: (R)-reticuline + NADP+ = 1,2-dehydroreticuline + H+ + NADPH.